{
  "gene": "UniProtKB:P21817",
  "gene_symbol": "RYR1",
  "term_label": "release of sequestered calcium ion into cytosol by sarcoplasmic reticulum",
  "gene_name": "Ryanodine receptor 1",
  "term_id": "GO:0014808"
}